{
  "gene_symbol": "ERGIC2",
  "term_id": "GO:0006888",
  "gene": "UniProtKB:Q96RQ1",
  "gene_name": "Endoplasmic reticulum-Golgi intermediate compartment protein 2",
  "term_label": "endoplasmic reticulum to Golgi vesicle-mediated transport"
}